{
  "term_label": "Unknown molecular function",
  "gene": "UniProtKB:Q9H814",
  "gene_name": "Phosphorylated adapter RNA export protein",
  "gene_symbol": "PHAX",
  "term_id": "UNKNOWN:0001"
}